nitrogen catabolite regulation of transcription [GO:0090293] (biological process) Relationships: is a type of regulation of DNA-templated transcription [GO:0006355]; is a type of regulation of nitrogen utilization [GO:0006808]; is a type of cellular response to nutrient [GO:0031670] Also known as: regulation of transcription by nitrogen catabolites References: PMID:19104072 Sources: GOC:mah, GOC:rb Definition: A transcription regulation process in which the presence of one nitrogen source leads to the modulation of the frequency, rate, or extent of transcription of specific genes involved in the metabolism of other nitrogen sources. Subtypes: nitrogen catabolite regulation of transcription from RNA polymerase II promoter [GO:0001079], nitrogen catabolite activation of transcription [GO:0090294], nitrogen catabolite repression of transcription [GO:0090295]